{
  "gene_symbol": "CNTN1",
  "term_label": "plasma membrane",
  "gene_name": "Contactin-1",
  "term_id": "GO:0005886",
  "gene": "UniProtKB:Q12860"
}